{
  "term_label": "memory",
  "term_id": "GO:0007613",
  "gene": "UniProtKB:Q9NQ66",
  "gene_name": "1-phosphatidylinositol 4,5-bisphosphate phosphodiesterase beta-1",
  "gene_symbol": "PLCB1"
}